positive regulation of erythrocyte enucleation [GO:0061931] (biological process) Definition: Any process that increases the frequency, rate or extent of erythrocyte enucleation. References: PMID:25241935 Relationships: is_a positive regulation of cellular component organization [GO:0051130]; is a type of regulation of erythrocyte enucleation [GO:0061930]; positively regulates erythrocyte enucleation [GO:0043131]